tetracyclic triterpenoid biosynthetic process [GO:0010686] (biological process) Sources: GOC:tair_curators Relationships: is a type of triterpenoid biosynthetic process [GO:0016104] Definition: The chemical reactions and pathways resulting in the formation of tetracyclic triterpenoid compounds, terpenoids with six isoprene units and 4 carbon rings. Also known as: tetracyclic triterpenoid biosynthesis Subtypes: (17Z)-protosta-17(20),24-dien-3beta-ol biosynthetic process [GO:1900581]